{
  "gene_name": "Epididymal secretory protein E3-beta",
  "term_label": "Unknown cellular component",
  "gene_symbol": "EDDM3B",
  "term_id": "UNKNOWN:0003",
  "gene": "UniProtKB:P56851"
}